regulation of Golgi organization [GO:1903358] (biological process) Relationships: is a type of GO:0033043; regulates Golgi organization [GO:0007030] Subtypes: GO:0090170, regulation of vesicle fusion with Golgi apparatus [GO:0106214] Definition: Any process that modulates the frequency, rate or extent of Golgi organization. Also known as: regulation of Golgi organisation, regulation of Golgi organization and biogenesis References: PMID:17562788 Sources: GOC:TermGenie, GOC:als, GO_REF:0000058